{
  "gene_name": "Protein shisa-like-2B",
  "term_id": "UNKNOWN:0003",
  "gene_symbol": "SHISAL2B",
  "term_label": "Unknown cellular component",
  "gene": "UniProtKB:A6NKW6"
}